2,4'-dihydroxyacetophenone dioxygenase activity [GO:0047073] (molecular function) Also known as: (4-hydroxybenzoyl)methanol oxygenase activity, 2,4'-dihydroxyacetophenone oxidoreductase (C-C-bond-cleaving) Definition: Catalysis of the reaction: 2,4'-dihydroxyacetophenone + O2 = 4-hydroxybenzoate + formate + 2 H+. Sources: EC:1.13.11.41, RHEA:24416 Relationships: is a type of oxidoreductase activity, acting on single donors with incorporation of molecular oxygen, incorporation of two atoms of oxygen [GO:0016702]